{
  "term_label": "proteasome-mediated ubiquitin-dependent protein catabolic process",
  "term_id": "GO:0043161",
  "gene": "UniProtKB:A0A0G2JMD5",
  "gene_symbol": "PRAMEF33",
  "gene_name": "PRAME family member 33"
}